{
  "term_id": "GO:0060271",
  "term_label": "cilium assembly",
  "gene_name": "Bardet-Biedl syndrome 4 protein",
  "gene_symbol": "BBS4",
  "gene": "UniProtKB:Q96RK4"
}